trichoblast fate specification [GO:0010057] (biological process) Sources: GOC:tb Relationships: is a type of plant epidermal cell fate specification [GO:0090628]; is part of trichoblast differentiation [GO:0010054] Regulation: regulated by GO:0010061; negatively regulated by negative regulation of trichoblast fate specification [GO:0010062]; positively regulated by GO:0010063 Definition: The process involved in the specification of a trichoblast.